floral organ morphogenesis [GO:0048444] (biological process) Subtypes: carpel morphogenesis [GO:0048445], petal morphogenesis [GO:0048446], sepal morphogenesis [GO:0048447], stamen morphogenesis [GO:0048448], floral organ structural organization [GO:0048450], anther morphogenesis [GO:0048654] Sources: GOC:PO_curators, GOC:go_curators, PO:0025395 Definition: The process in which the anatomical structures of the floral organ are generated and organized. Relationships: is_a developmental process involved in reproduction [GO:0003006]; is a type of GO:0090697; is part of floral organ development [GO:0048437]